{
  "gene": "UniProtKB:Q2WGJ8",
  "term_id": "UNKNOWN:0002",
  "gene_name": "Cation channel sperm-associated auxiliary subunit TMEM249",
  "term_label": "Unknown biological process",
  "gene_symbol": "TMEM249"
}